{
  "gene_symbol": "XPO7",
  "gene": "UniProtKB:Q9UIA9",
  "term_label": "cytoplasm",
  "gene_name": "Exportin-7",
  "term_id": "GO:0005737"
}